viral transcriptional complex [GO:0019036] (cellular component) Sources: ISBN:0781718325 Relationships: is a type of protein-containing complex [GO:0032991] Definition: Specific locations and structures in the virus infected cell involved in transcribing the viral genome.